{
  "gene_symbol": "SEMA4G",
  "term_id": "GO:0050919",
  "gene_name": "Semaphorin-4G",
  "gene": "UniProtKB:Q9NTN9",
  "term_label": "negative chemotaxis"
}